{
  "term_id": "GO:0034976",
  "gene_symbol": "TMEM259",
  "gene": "UniProtKB:Q4ZIN3",
  "gene_name": "Membralin",
  "term_label": "response to endoplasmic reticulum stress"
}